{
  "gene": "UniProtKB:Q08AM6",
  "term_label": "PAS complex",
  "gene_name": "Protein VAC14 homolog",
  "gene_symbol": "VAC14",
  "term_id": "GO:0070772"
}